{
  "term_label": "membrane",
  "term_id": "GO:0016020",
  "gene_symbol": "PLPP7",
  "gene": "UniProtKB:Q8NBV4",
  "gene_name": "Inactive phospholipid phosphatase 7"
}